cardiac cell development [GO:0055006] (biological process) Sources: GOC:devbiol Definition: The process whose specific outcome is the progression of a cardiac cell over time, from its formation to the mature state. A cardiac cell is a cell that will form part of the cardiac organ of an individual. Relationships: is a type of cell development [GO:0048468]; is part of GO:0035051 Subtypes: cardiac muscle cell development [GO:0055013], GO:0060933, cardiac fibroblast cell development [GO:0060936], GO:0060948, GO:0060952, endocardial cell development [GO:0060958], GO:0060959, endocardial cushion cell development [GO:0061444] Also known as: cardiocyte development, heart cell development